postsynaptic actin cytoskeleton [GO:0098871] (cellular component) Subtypes: actin cytoskeleton of dendritic spine [GO:0098938] Relationships: is a type of actin cytoskeleton [GO:0015629]; is a type of postsynaptic cytoskeleton [GO:0099571] Sources: GOC:dos Definition: The actin cytoskeleton that is part of a postsynapse.